response to Gram-negative bacterium [GO:0140460] (biological process) Definition: Any process that results in a change in state or activity of a cell or an organism (in terms of movement, secretion, enzyme production, gene expression, etc.) as a result of a stimulus from a Gram-negative bacterium. References: PMID:23664307 Relationships: is a type of response to bacterium [GO:0009617]